asperfuranone biosynthetic process [GO:1900554] (biological process) Also known as: asperfuranone anabolism, asperfuranone biosynthesis, asperfuranone formation, asperfuranone synthesis Sources: GOC:TermGenie, GOC:di Relationships: is a type of GO:0030639; is_a diol biosynthetic process [GO:0034312]; is a type of GO:0042181; is a type of GO:1902645; is a type of secondary alcohol biosynthetic process [GO:1902653] Definition: The chemical reactions and pathways resulting in the formation of asperfuranone. Regulation: regulated by regulation of asperfuranone biosynthetic process [GO:1900637]; negatively regulated by GO:1900638; positively regulated by GO:1900639